regulation of biological process involved in symbiotic interaction [GO:0043903] (biological process) Relationships: is a type of regulation of biological process [GO:0050789]; regulates biological process involved in symbiotic interaction [GO:0044403] Also known as: regulation of interspecies interactions between organisms, regulation of symbiotic process, regulation of symbiosis, encompassing mutualism through parasitism Sources: GOC:jl Subtypes: modulation by symbiont of entry into host [GO:0052372], regulation of neutrophil mediated killing of symbiont cell [GO:0070949], GO:0075045, positive regulation of transepithelial migration of symbiont in host [GO:0140471], regulation of single-species biofilm formation in or on host organism [GO:1900228], regulation of intracellular transport of viral material [GO:1901252], regulation of receptor-mediated virion attachment to host cell [GO:1902734], regulation of transformation of host cell by virus [GO:1904187] Definition: Any process that modulates the frequency, rate or extent of symbiosis, an interaction between two organisms living together in more or less intimate association. Note: regulation of interspecies interactions between organisms